{
  "gene": "UniProtKB:Q99996",
  "term_label": "potassium channel regulator activity",
  "gene_name": "A-kinase anchor protein 9",
  "gene_symbol": "AKAP9",
  "term_id": "GO:0015459"
}